{
  "gene": "UniProtKB:P62807",
  "gene_name": "Histone H2B type 1-C_E_F_G_I",
  "gene_symbol": "H2BC10",
  "term_label": "structural constituent of chromatin",
  "term_id": "GO:0030527"
}